{
  "term_id": "UNKNOWN:0002",
  "gene_symbol": "TEX13A",
  "term_label": "Unknown biological process",
  "gene_name": "Testis-expressed protein 13A",
  "gene": "UniProtKB:Q9BXU3"
}